(-)-isopiperitenone reductase activity [GO:0052581] (molecular function) Also known as: (+)-cis-isopulegone:NADP+ oxidoreductase activity Relationships: is a type of enone reductase activity [GO:0035671] Sources: EC:1.3.1.82, RHEA:25649 Definition: Catalysis of the reaction: (6R)-isoperitenone + H+ + NADPH = (2R,5R)-isopulegone + NADP+.